{
  "term_label": "cytoplasm",
  "term_id": "GO:0005737",
  "gene": "UniProtKB:Q15149",
  "gene_symbol": "PLEC",
  "gene_name": "Plectin"
}